{
  "gene_symbol": "MECR",
  "term_label": "mitochondrion",
  "gene": "UniProtKB:Q9BV79",
  "term_id": "GO:0005739",
  "gene_name": "Enoyl-[acyl-carrier-protein] reductase, mitochondrial"
}